{
  "gene_symbol": "USP26",
  "gene_name": "Ubiquitin carboxyl-terminal hydrolase 26",
  "gene": "UniProtKB:Q9BXU7",
  "term_label": "regulation of protein stability",
  "term_id": "GO:0031647"
}